{
  "term_id": "GO:0098553",
  "gene_symbol": "SPPL2A",
  "gene": "UniProtKB:Q8TCT8",
  "gene_name": "Signal peptide peptidase-like 2A",
  "term_label": "lumenal side of endoplasmic reticulum membrane"
}